{
  "gene": "UniProtKB:Q8TCN5",
  "term_label": "nucleus",
  "gene_name": "Zinc finger protein 507",
  "term_id": "GO:0005634",
  "gene_symbol": "ZNF507"
}